(S)-coclaurine-N-methyltransferase activity [GO:0030794] (molecular function) Relationships: is a type of S-adenosylmethionine-dependent methyltransferase activity [GO:0008757] Also known as: S-adenosyl-L-methionine:(S)-coclaurine-N-methyltransferase activity Sources: EC:2.1.1.140 Definition: Catalysis of the reaction: S-adenosyl-L-methionine + (S)-coclaurine = S-adenosyl-L-homocysteine + (S)-N-methylcoclaurine.